{
  "gene": "UniProtKB:A6NGB9",
  "term_label": "early endosome",
  "gene_symbol": "WIPF3",
  "gene_name": "WAS_WASL-interacting protein family member 3",
  "term_id": "GO:0005769"
}